{
  "term_id": "UNKNOWN:0003",
  "term_label": "Unknown cellular component",
  "gene_name": "SCAN domain-containing protein 1",
  "gene": "UniProtKB:P57086",
  "gene_symbol": "SCAND1"
}